{
  "term_id": "GO:0005615",
  "term_label": "extracellular space",
  "gene": "UniProtKB:P05121",
  "gene_symbol": "SERPINE1",
  "gene_name": "Plasminogen activator inhibitor 1"
}